{
  "gene_symbol": "ACO2",
  "term_id": "GO:0005829",
  "gene_name": "Aconitate hydratase, mitochondrial",
  "term_label": "cytosol",
  "gene": "UniProtKB:Q99798"
}